{
  "gene_name": "Cleavage and polyadenylation specificity factor subunit 5",
  "gene_symbol": "NUDT21",
  "gene": "UniProtKB:O43809",
  "term_label": "mRNA processing",
  "term_id": "GO:0006397"
}